{
  "term_id": "GO:0008023",
  "gene_symbol": "ELL2",
  "gene": "UniProtKB:O00472",
  "gene_name": "RNA polymerase II elongation factor ELL2",
  "term_label": "transcription elongation factor complex"
}